negative regulation of cholangiocyte proliferation [GO:1904055] (biological process) Relationships: is a type of GO:0050680; is a type of regulation of cholangiocyte proliferation [GO:1904054]; negatively regulates GO:1990705 Also known as: down regulation of cholangiocyte proliferation, down regulation of hepatoblast proliferation, down-regulation of cholangiocyte proliferation, down-regulation of hepatoblast proliferation, downregulation of cholangiocyte proliferation, downregulation of hepatoblast proliferation, negative regulation of hepatoblast proliferation, inhibition of cholangiocyte proliferation, inhibition of hepatoblast proliferation Definition: Any process that stops, prevents or reduces the frequency, rate or extent of cholangiocyte proliferation. References: PMID:24434010 Sources: GOC:TermGenie, GO_REF:0000058